{
  "gene": "UniProtKB:Q14123",
  "term_label": "calmodulin-activated 3',5'-cyclic-GMP phosphodiesterase activity",
  "gene_name": "Dual specificity calcium_calmodulin-dependent 3',5'-cyclic nucleotide phosphodiesterase 1C",
  "term_id": "GO:0048101",
  "gene_symbol": "PDE1C"
}